bone remodeling [GO:0046849] (biological process) Sources: GOC:curators Relationships: is a type of tissue remodeling [GO:0048771] Also known as: bone remodelling Regulation: regulated by regulation of bone remodeling [GO:0046850]; negatively regulated by negative regulation of bone remodeling [GO:0046851]; positively regulated by positive regulation of bone remodeling [GO:0046852] Definition: The continuous turnover of bone matrix and mineral that involves first, an increase in resorption (osteoclastic activity) and later, reactive bone formation (osteoblastic activity). The process of bone remodeling takes place in the adult skeleton at discrete foci. The process ensures the mechanical integrity of the skeleton throughout life and plays an important role in calcium homeostasis. An imbalance in the regulation of bone resorption and bone formation results in many of the metabolic bone diseases, such as osteoporosis.